{
  "term_id": "GO:0050911",
  "term_label": "detection of chemical stimulus involved in sensory perception of smell",
  "gene": "UniProtKB:Q8NGY9",
  "gene_symbol": "OR2L8",
  "gene_name": "Olfactory receptor 2L8"
}